{
  "gene": "UniProtKB:P22894",
  "gene_name": "Neutrophil collagenase",
  "term_label": "collagen catabolic process",
  "gene_symbol": "MMP8",
  "term_id": "GO:0030574"
}